regulation of RNA stability [GO:0043487] (biological process) Subtypes: regulation of tRNA stability [GO:0036415], regulation of mRNA stability [GO:0043488], RNA stabilization [GO:0043489], regulation of rRNA stability [GO:0044357], RNA destabilization [GO:0050779] Definition: Any process that modulates the propensity of RNA molecules to degradation. Includes processes that both stabilize and destabilize RNAs. Relationships: is a type of regulation of catabolic process [GO:0009894]; is a type of GO:0010608; is a type of GO:0051252; is a type of regulation of biological quality [GO:0065008]; regulates RNA catabolic process [GO:0006401] Sources: GOC:jl